{
  "term_label": "Unknown biological process",
  "gene": "UniProtKB:Q96RD1",
  "term_id": "UNKNOWN:0002",
  "gene_name": "Olfactory receptor 6C1",
  "gene_symbol": "OR6C1"
}